{
  "term_id": "GO:0051256",
  "gene": "UniProtKB:Q9H0H5",
  "gene_symbol": "RACGAP1",
  "gene_name": "Rac GTPase-activating protein 1",
  "term_label": "mitotic spindle midzone assembly"
}